{
  "gene": "UniProtKB:P07949",
  "gene_name": "Proto-oncogene tyrosine-protein kinase receptor Ret",
  "term_label": "receptor complex",
  "term_id": "GO:0043235",
  "gene_symbol": "RET"
}